{
  "term_id": "UNKNOWN:0003",
  "term_label": "Unknown cellular component",
  "gene": "UniProtKB:A0A096LPG2",
  "gene_name": "Uncharacterized protein",
  "gene_symbol": "A0A096LPG2"
}